{
  "gene": "UniProtKB:O60684",
  "gene_symbol": "KPNA6",
  "term_id": "GO:0005634",
  "term_label": "nucleus",
  "gene_name": "Importin subunit alpha-7"
}